{
  "gene": "UniProtKB:Q9GZM3",
  "gene_name": "DNA-directed RNA polymerase II subunit RPB11-b1",
  "term_id": "GO:0006366",
  "term_label": "transcription by RNA polymerase II",
  "gene_symbol": "POLR2J2"
}